regulation of fast-twitch skeletal muscle fiber contraction [GO:0031446] (BP) Definition: Any process that modulates the frequency, rate or extent of fast-twitch skeletal muscle contraction. Also known as: regulation of fast-twitch skeletal muscle contraction Subtypes: GO:0031447, positive regulation of fast-twitch skeletal muscle fiber contraction [GO:0031448] Sources: GOC:dph, GOC:ef, GOC:mah, GOC:mtg_muscle, GOC:tb Relationships: is a type of GO:0014724; regulates fast-twitch skeletal muscle fiber contraction [GO:0031443]